{
  "gene": "UniProtKB:Q9HCC0",
  "gene_symbol": "MCCC2",
  "term_id": "GO:1905202",
  "term_label": "methylcrotonoyl-CoA carboxylase complex",
  "gene_name": "Methylcrotonoyl-CoA carboxylase beta chain, mitochondrial"
}